positive regulation of pseudohyphal growth by positive regulation of transcription from RNA polymerase II promoter [GO:1900461] (biological process) Relationships: is a type of GO:0045944; is a type of positive regulation of pseudohyphal growth [GO:2000222] References: PMID:11046133, PMID:8710886, PMID:9987114 Sources: GOC:TermGenie, GOC:dgf Definition: Any process that activates or increases the frequency, rate or extent of pseudohyphal growth by activating or increasing the frequency, rate or extent of transcription from an RNA polymerase II promoter.